{
  "gene_symbol": "HTATIP2",
  "term_id": "GO:0004674",
  "gene_name": "Oxidoreductase HTATIP2",
  "gene": "UniProtKB:Q9BUP3",
  "term_label": "protein serine/threonine kinase activity"
}